{
  "term_id": "GO:0004252",
  "term_label": "serine-type endopeptidase activity",
  "gene_name": "Complement factor D",
  "gene": "UniProtKB:P00746",
  "gene_symbol": "CFD"
}